epithelial cell fate commitment [GO:0072148] (biological process) Definition: The process in which the developmental fate of a cell becomes restricted such that it will develop into an epithelial cell. Relationships: is a type of cell fate commitment [GO:0045165]; is part of GO:0030855 Subtypes: pancreatic A cell fate commitment [GO:0003326], GO:0003327, pancreatic D cell fate commitment [GO:0003328], pancreatic PP cell fate commitment [GO:0003329], GO:0035027, Sertoli cell fate commitment [GO:0060010], granulosa cell fate commitment [GO:0060015], endothelial cell fate commitment [GO:0060839], glomerular parietal epithelial cell fate commitment [GO:0072147], podocyte cell fate commitment [GO:0072149] Sources: GOC:mtg_kidney_jan10